{
  "term_id": "UNKNOWN:0002",
  "gene_name": "UPF0488 protein C8orf33",
  "gene": "UniProtKB:Q9H7E9",
  "term_label": "Unknown biological process",
  "gene_symbol": "C8orf33"
}